{
  "term_label": "Golgi apparatus",
  "term_id": "GO:0005794",
  "gene": "UniProtKB:Q9Y287",
  "gene_symbol": "ITM2B",
  "gene_name": "Integral membrane protein 2B"
}